positive regulation of activated T cell proliferation [GO:0042104] (biological process) Relationships: is a type of positive regulation of T cell proliferation [GO:0042102]; is a type of regulation of activated T cell proliferation [GO:0046006]; positively regulates GO:0050798 Definition: Any process that activates or increases the rate or extent of activated T cell proliferation. Sources: GOC:jl Also known as: positive regulation of activated T lymphocyte proliferation, positive regulation of activated T-cell proliferation, positive regulation of activated T-lymphocyte proliferation, up regulation of activated T cell proliferation, up-regulation of activated T cell proliferation, upregulation of activated T cell proliferation, activation of activated T cell proliferation, stimulation of activated T cell proliferation